pyrimidine nucleoside triphosphate biosynthetic process [GO:0009148] (biological process) Also known as: pyrimidine nucleoside triphosphate anabolism, pyrimidine nucleoside triphosphate biosynthesis, pyrimidine nucleoside triphosphate formation, pyrimidine nucleoside triphosphate synthesis Subtypes: GO:0009209, pyrimidine deoxyribonucleoside triphosphate biosynthetic process [GO:0009212] Sources: GOC:go_curators, ISBN:0198506732 Definition: The chemical reactions and pathways resulting in the formation of pyrimidine nucleoside triphosphate, a compound consisting of a pyrimidine base linked to a ribose or deoxyribose sugar esterified with triphosphate on the sugar. Relationships: is a type of nucleoside triphosphate biosynthetic process [GO:0009142]; is a type of pyrimidine nucleoside triphosphate metabolic process [GO:0009147]